10-hydroxygeranial oxidoreductase activity [GO:0102968] (molecular function) Relationships: is a type of oxidoreductase activity, acting on the CH-OH group of donors, NAD or NADP as acceptor [GO:0016616] Sources: GOC:pz, RHEA:32611 Definition: Catalysis of the reaction: (6E)-8-hydroxygeranial + NADP = (6E)-8-oxogeranial + NADPH + H+.